{
  "gene_name": "CST complex subunit TEN1",
  "term_id": "GO:1990879",
  "gene": "UniProtKB:Q86WV5",
  "term_label": "CST complex",
  "gene_symbol": "TEN1"
}